{
  "term_label": "Unknown cellular component",
  "gene_name": "V-set and immunoglobulin domain-containing protein 10-like",
  "gene": "UniProtKB:Q86VR7",
  "gene_symbol": "VSIG10L",
  "term_id": "UNKNOWN:0003"
}